actin rod assembly [GO:0031247] (biological process) References: PMID:14706699 Sources: GOC:pg Definition: The assembly of actin rods, a cellular structure consisting of parallel, hexagonally arranged actin tubules. Relationships: is a type of actin filament bundle assembly [GO:0051017] Also known as: actin rod formation